{
  "gene_symbol": "CD74",
  "term_label": "MHC class II protein binding",
  "term_id": "GO:0042289",
  "gene_name": "HLA class II histocompatibility antigen gamma chain",
  "gene": "UniProtKB:P04233"
}